ribitol biosynthetic process [GO:0046362] (biological process) Relationships: is a type of pentitol biosynthetic process [GO:0019526] Also known as: ribitol anabolism, ribitol biosynthesis, ribitol formation, ribitol synthesis Sources: ISBN:0198506732 Definition: The chemical reactions and pathways resulting in the formation of ribitol, a pentitol derived formally by reduction of the -CHO group of either D- or L-ribose.